{
  "term_label": "Unknown biological process",
  "term_id": "UNKNOWN:0002",
  "gene": "UniProtKB:A6NDL8",
  "gene_symbol": "OR6C68",
  "gene_name": "Olfactory receptor 6C68"
}